{
  "gene_name": "Neuronal acetylcholine receptor subunit alpha-2",
  "term_label": "plasma membrane",
  "gene_symbol": "CHRNA2",
  "gene": "UniProtKB:Q15822",
  "term_id": "GO:0005886"
}